animal organ maturation [GO:0048799] (biological process) Definition: A developmental process, independent of morphogenetic (shape) change, that is required for an animal organ to attain its fully functional state. An organ is a tissue or set of tissues that work together to perform a specific function or functions. Subtypes: ureter maturation [GO:0035799], swim bladder maturation [GO:0048796], bone maturation [GO:0070977], GO:0072120 Relationships: is a type of GO:0071695; is part of animal organ development [GO:0048513] Sources: GOC:curators